{
  "gene_symbol": "FAR1",
  "gene": "UniProtKB:Q8WVX9",
  "term_label": "long-chain fatty-acyl-CoA metabolic process",
  "term_id": "GO:0035336",
  "gene_name": "Fatty acyl-CoA reductase 1"
}